{
  "gene_name": "Protein FAM133B",
  "gene": "UniProtKB:Q5BKY9",
  "term_id": "UNKNOWN:0003",
  "gene_symbol": "FAM133B",
  "term_label": "Unknown cellular component"
}